{
  "gene_name": "Olfactory receptor 2V2",
  "term_id": "GO:0005886",
  "gene_symbol": "OR2V2",
  "gene": "UniProtKB:Q96R30",
  "term_label": "plasma membrane"
}